{
  "gene_symbol": "TRABD2B",
  "gene_name": "Metalloprotease TIKI2",
  "gene": "UniProtKB:A6NFA1",
  "term_label": "organelle membrane",
  "term_id": "GO:0031090"
}